phosphatidylinositol phosphate 4-phosphatase activity [GO:0034596] (MF) Sources: GOC:mah Definition: Catalysis of the removal of the 4-phosphate group of a phosphatidylinositol phosphate. Subtypes: phosphatidylinositol-3,4-bisphosphate 4-phosphatase activity [GO:0016316], GO:0034597, GO:0043812 Also known as: PI(4)P-phosphatase activity, PI4P-phosphatase activity, PtdIns4P-phosphatase activity, phosphoinositide 4-phosphatase activity, inositol 4-phosphatase Relationships: is a type of phosphatidylinositol phosphate phosphatase activity [GO:0052866]